{
  "term_id": "UNKNOWN:0003",
  "term_label": "Unknown cellular component",
  "gene": "UniProtKB:Q86UY8",
  "gene_name": "5'-nucleotidase domain-containing protein 3",
  "gene_symbol": "NT5DC3"
}